{
  "term_id": "UNKNOWN:0001",
  "gene_symbol": "WDR54",
  "term_label": "Unknown molecular function",
  "gene": "UniProtKB:Q9H977",
  "gene_name": "WD repeat-containing protein 54"
}